positive regulation of mRNA splicing, via spliceosome [GO:0048026] (BP) Subtypes: GO:1905746 Sources: GOC:jid Also known as: positive regulation of pre-mRNA splicing, positive regulation of nuclear mRNA splicing, via spliceosome, up regulation of nuclear mRNA splicing, via spliceosome, up-regulation of nuclear mRNA splicing, via spliceosome, upregulation of nuclear mRNA splicing, via spliceosome, activation of nuclear mRNA splicing via U2-type spliceosome, activation of nuclear mRNA splicing, via spliceosome, positive regulation of nuclear mRNA splicing via U2-type spliceosome, stimulation of nuclear mRNA splicing via U2-type spliceosome, stimulation of nuclear mRNA splicing, via spliceosome, up regulation of nuclear mRNA splicing via U2-type spliceosome, up-regulation of nuclear mRNA splicing via U2-type spliceosome, upregulation of nuclear mRNA splicing via U2-type spliceosome Relationships: is a type of positive regulation of RNA splicing [GO:0033120]; is a type of regulation of mRNA splicing, via spliceosome [GO:0048024]; is_a positive regulation of mRNA processing [GO:0050685]; positively regulates mRNA splicing, via spliceosome [GO:0000398] Definition: Any process that activates or increases the rate or extent of mRNA splicing via a spliceosomal mechanism.